positive regulation of cardiac muscle cell apoptotic process [GO:0010666] (BP) Sources: GOC:dph, GOC:mtg_apoptosis, GOC:tb Relationships: is a type of GO:0010663; is a type of regulation of cardiac muscle cell apoptotic process [GO:0010665]; positively regulates cardiac muscle cell apoptotic process [GO:0010659] Also known as: positive regulation of cardiac muscle cell apoptosis Definition: Any process that increases the rate or extent of cardiac cell apoptotic process, a form of programmed cell death induced by external or internal signals that trigger the activity of proteolytic caspases whose actions dismantle a cardiac muscle cell and result in its death.